{
  "gene_name": "Cyclin-dependent kinase inhibitor 1B",
  "term_label": "nucleus",
  "gene_symbol": "CDKN1B",
  "term_id": "GO:0005634",
  "gene": "UniProtKB:P46527"
}